{
  "gene_name": "Mitochondrial enolase superfamily member 1",
  "gene_symbol": "ENOSF1",
  "term_label": "Unknown cellular component",
  "gene": "UniProtKB:Q7L5Y1",
  "term_id": "UNKNOWN:0003"
}